{
  "term_id": "UNKNOWN:0002",
  "gene": "UniProtKB:A0A6Q8PHS2",
  "gene_symbol": "A0A6Q8PHS2",
  "term_label": "Unknown biological process",
  "gene_name": "Uncharacterized protein"
}